{
  "term_id": "GO:0007043",
  "gene_symbol": "CDH20",
  "term_label": "cell-cell junction assembly",
  "gene": "UniProtKB:Q9HBT6",
  "gene_name": "Cadherin-20"
}